{
  "gene_symbol": "GOLPH3L",
  "gene": "UniProtKB:Q9H4A5",
  "gene_name": "Golgi phosphoprotein 3-like",
  "term_id": "GO:0031985",
  "term_label": "Golgi cisterna"
}